{
  "gene": "UniProtKB:P41002",
  "gene_name": "Cyclin-F",
  "gene_symbol": "CCNF",
  "term_id": "GO:0000307",
  "term_label": "cyclin-dependent protein kinase holoenzyme complex"
}